{
  "term_id": "GO:0007166",
  "gene_name": "X-linked interleukin-1 receptor accessory protein-like 2",
  "gene": "UniProtKB:Q9NP60",
  "gene_symbol": "IL1RAPL2",
  "term_label": "cell surface receptor signaling pathway"
}